epidermal growth factor receptor signaling pathway involved in lung development [GO:0060507] (biological process) Also known as: epidermal growth factor receptor signalling pathway involved in lung development Relationships: is a type of epidermal growth factor receptor signaling pathway [GO:0007173]; is part of cell-cell signaling involved in lung development [GO:0060495] Sources: GOC:dph, GOC:mtg_lung Definition: The series of molecular signals generated as a consequence of an epidermal growth factor-type receptor binding to one of its physiological ligands. This process contributes to lung development.